{
  "gene": "UniProtKB:A0A1B0GUA7",
  "gene_name": "Testis-expressed protein 51",
  "gene_symbol": "TEX51",
  "term_label": "Unknown cellular component",
  "term_id": "UNKNOWN:0003"
}